{
  "gene_name": "Sorting nexin-25",
  "gene": "UniProtKB:Q9H3E2",
  "gene_symbol": "SNX25",
  "term_label": "endosome",
  "term_id": "GO:0005768"
}